{
  "term_id": "GO:0006357",
  "gene_name": "POU domain, class 4, transcription factor 3",
  "gene": "UniProtKB:Q15319",
  "gene_symbol": "POU4F3",
  "term_label": "regulation of transcription by RNA polymerase II"
}